copulation [GO:0007620] (biological process) Definition: The act of sexual union between male and female, involving the transfer of sperm. Sources: ISBN:0721662544 Relationships: is a type of mating behavior [GO:0007617]